{
  "term_label": "mRNA 3'-UTR binding",
  "term_id": "GO:0003730",
  "gene": "UniProtKB:Q86SH2",
  "gene_name": "Zygote arrest protein 1",
  "gene_symbol": "ZAR1"
}